{
  "term_id": "GO:0042060",
  "gene_symbol": "DCBLD2",
  "gene": "UniProtKB:Q96PD2",
  "gene_name": "Discoidin, CUB and LCCL domain-containing protein 2",
  "term_label": "wound healing"
}